{
  "gene_symbol": "PNAS-138",
  "term_label": "Unknown biological process",
  "term_id": "UNKNOWN:0002",
  "gene_name": "Putative uncharacterized protein PNAS-138",
  "gene": "UniProtKB:Q9BZS9"
}